metanephric mesenchyme development [GO:0072075] (biological process) Sources: GOC:mtg_kidney_jan10 Subtypes: metanephric cap development [GO:0072185] Definition: The biological process whose specific outcome is the progression of a metanephric mesenchyme from an initial condition to its mature state. This process begins with the formation of metanephric mesenchyme and ends with the mature structure. Metanephric mesenchyme is the tissue made up of loosely connected mesenchymal cells in the metanephros. Relationships: is a type of kidney mesenchyme development [GO:0072074]; is part of metanephros development [GO:0001656]